{
  "term_id": "UNKNOWN:0002",
  "gene_name": "Coiled-coil domain-containing protein 187",
  "term_label": "Unknown biological process",
  "gene_symbol": "CCDC187",
  "gene": "UniProtKB:A0A096LP49"
}